{
  "term_label": "tubulin binding",
  "gene_symbol": "STMN1",
  "gene": "UniProtKB:P16949",
  "term_id": "GO:0015631",
  "gene_name": "Stathmin"
}